{
  "gene_symbol": "RNF213",
  "term_label": "sprouting angiogenesis",
  "gene_name": "E3 ubiquitin-protein ligase RNF213",
  "gene": "UniProtKB:Q63HN8",
  "term_id": "GO:0002040"
}